{
  "term_label": "nucleosome",
  "gene_symbol": "H2AC1",
  "gene": "UniProtKB:Q96QV6",
  "term_id": "GO:0000786",
  "gene_name": "Histone H2A type 1-A"
}